{
  "gene_name": "Dynein assembly factor with WDR repeat domains 1",
  "term_id": "GO:0000209",
  "gene_symbol": "DAW1",
  "term_label": "protein polyubiquitination",
  "gene": "UniProtKB:Q8N136"
}